vesicle targeting, inter-Golgi cisterna [GO:0048204] (biological process) References: PMID:10219233 Sources: GOC:jid, GOC:mah, ISBN:0716731363 Definition: The process in which vesicles are directed to specific destination membranes during transport from one Golgi cisterna to another. Also known as: inter-Golgi cisterna targeting Relationships: is a type of vesicle targeting, to, from or within Golgi [GO:0048199]; is part of GO:0048219